{
  "term_label": "U2 snRNP",
  "gene_name": "Splicing factor 3B subunit 4",
  "term_id": "GO:0005686",
  "gene": "UniProtKB:Q15427",
  "gene_symbol": "SF3B4"
}